{
  "gene_name": "Putative nuclear envelope pore membrane protein POM 121B",
  "gene": "UniProtKB:A6NF01",
  "term_label": "nuclear pore",
  "term_id": "GO:0005643",
  "gene_symbol": "POM121B"
}